negative regulation of T cell cytokine production [GO:0002725] (biological process) Subtypes: negative regulation of T-helper 2 cell cytokine production [GO:2000552], negative regulation of T-helper 1 cell cytokine production [GO:2000555] Relationships: is a type of negative regulation of T cell mediated immunity [GO:0002710]; is a type of GO:0002719; is a type of GO:0002724; negatively regulates T cell cytokine production [GO:0002369] Definition: Any process that stops, prevents, or reduces the frequency, rate, or extent of T cell cytokine production. Also known as: down regulation of T cell cytokine production, down-regulation of T cell cytokine production, downregulation of T cell cytokine production, negative regulation of T lymphocyte cytokine production, negative regulation of T-cell cytokine production, negative regulation of T-lymphocyte cytokine production, inhibition of T cell cytokine production Sources: GOC:add